{
  "gene_symbol": "C12orf56",
  "term_id": "UNKNOWN:0001",
  "term_label": "Unknown molecular function",
  "gene_name": "Uncharacterized protein C12orf56",
  "gene": "UniProtKB:Q8IXR9"
}